{
  "gene": "UniProtKB:Q9BV97",
  "gene_name": "Zinc finger protein 747",
  "term_id": "GO:0000978",
  "term_label": "RNA polymerase II cis-regulatory region sequence-specific DNA binding",
  "gene_symbol": "ZNF747"
}